{
  "term_id": "UNKNOWN:0003",
  "gene": "UniProtKB:A0A0U1RRL7",
  "gene_symbol": "MMP24OS",
  "gene_name": "Protein MMP24OS",
  "term_label": "Unknown cellular component"
}